{
  "term_label": "nucleus",
  "gene": "UniProtKB:Q99460",
  "term_id": "GO:0005634",
  "gene_symbol": "PSMD1",
  "gene_name": "26S proteasome non-ATPase regulatory subunit 1"
}